{
  "term_id": "GO:0055085",
  "gene_symbol": "SLC13A5",
  "term_label": "transmembrane transport",
  "gene_name": "Na(+)_citrate cotransporter",
  "gene": "UniProtKB:Q86YT5"
}